{
  "term_id": "GO:0005737",
  "gene": "UniProtKB:Q9NZJ5",
  "gene_name": "Eukaryotic translation initiation factor 2-alpha kinase 3",
  "term_label": "cytoplasm",
  "gene_symbol": "EIF2AK3"
}